{
  "gene_name": "Sulfate anion transporter 1",
  "gene": "UniProtKB:Q9H2B4",
  "gene_symbol": "SLC26A1",
  "term_label": "sulfate transmembrane transporter activity",
  "term_id": "GO:0015116"
}